urea binding [GO:0033219] (molecular function) Sources: GOC:mah, ISBN:0198506732 Definition: Binding to urea, a water-soluble carboxamide with the structure H2N-CO-NH2. Relationships: is a type of amide binding [GO:0033218]; is a type of GO:0036094